regulation of Malpighian tubule size [GO:0035298] (biological process) Definition: Ensuring that a Malpighian tubule is the correct length and diameter. Subtypes: regulation of Malpighian tubule diameter [GO:0035297] Sources: GOC:bf Relationships: is a type of GO:0035150; is part of GO:0007443